{
  "term_id": "UNKNOWN:0002",
  "gene": "UniProtKB:Q69YL0",
  "term_label": "Unknown biological process",
  "gene_symbol": "NCBP2AS2",
  "gene_name": "Protein NCBP2AS2"
}